{
  "gene_name": "Coiled-coil domain-containing protein 159",
  "gene_symbol": "CCDC159",
  "term_label": "Unknown cellular component",
  "gene": "UniProtKB:P0C7I6",
  "term_id": "UNKNOWN:0003"
}